{
  "term_id": "UNKNOWN:0001",
  "term_label": "Unknown molecular function",
  "gene_symbol": "IGSF3",
  "gene_name": "Immunoglobulin superfamily member 3",
  "gene": "UniProtKB:O75054"
}